{
  "term_id": "GO:1904062",
  "gene_symbol": "NRBP2",
  "term_label": "regulation of monoatomic cation transmembrane transport",
  "gene_name": "Nuclear receptor-binding protein 2",
  "gene": "UniProtKB:Q9NSY0"
}